{
  "gene_name": "HAUS augmin-like complex subunit 2",
  "term_label": "centrosome cycle",
  "term_id": "GO:0007098",
  "gene_symbol": "HAUS2",
  "gene": "UniProtKB:Q9NVX0"
}